meiotic spindle assembly [GO:0090306] (biological process) Definition: The aggregation, arrangement and bonding together of a set of components to form the spindle that contributes to the process of meiosis. Sources: GOC:tb, GOC:vw Also known as: spindle assembly involved in meiosis Relationships: is a type of meiotic spindle organization [GO:0000212]; is_a spindle assembly [GO:0051225]; is part of meiotic chromosome segregation [GO:0045132] Subtypes: GO:0007053, spindle assembly involved in female meiosis [GO:0007056], GO:0140642